negative regulation of MDA-5 signaling pathway [GO:0039534] (biological process) Also known as: negative regulation of IFIH1 signaling pathway, negative regulation of MDA-5 signalling pathway, negative regulation of MDA5 signaling pathway, negative regulation of melanoma differentiation-associated gene 5 signaling pathway Relationships: is a type of negative regulation of cytoplasmic pattern recognition receptor signaling pathway [GO:0039532]; is a type of regulation of MDA-5 signaling pathway [GO:0039533]; negatively regulates MDA-5 signaling pathway [GO:0039530] Definition: Any process that stops, prevents, or reduces the frequency, rate or extent of the series of the MDA-5 signaling pathway. Sources: GOC:bf, GOC:jl